{
  "gene": "UniProtKB:Q9ULK2",
  "gene_symbol": "ATXN7L1",
  "term_id": "UNKNOWN:0002",
  "gene_name": "Ataxin-7-like protein 1",
  "term_label": "Unknown biological process"
}